{
  "gene": "UniProtKB:P01241",
  "term_id": "GO:0031667",
  "term_label": "response to nutrient levels",
  "gene_name": "Somatotropin",
  "gene_symbol": "GH1"
}